{
  "gene": "UniProtKB:Q86UQ4",
  "term_label": "lipid transporter activity",
  "gene_name": "ATP-binding cassette sub-family A member 13",
  "gene_symbol": "ABCA13",
  "term_id": "GO:0005319"
}